negative regulation of neutrophil aggregation [GO:2000429] (BP) Sources: GOC:BHF Definition: Any process that stops, prevents or reduces the frequency, rate or extent of neutrophil aggregation. Relationships: is a type of negative regulation of leukocyte cell-cell adhesion [GO:1903038]; is a type of GO:2000428; negatively regulates neutrophil aggregation [GO:0070488] Also known as: negative regulation of neutrocyte aggregation, negative regulation of neutrophil leucocyte aggregation, negative regulation of neutrophilic leukocyte aggregation